regulation of constitutive secretory pathway [GO:1903433] (biological process) Relationships: is a type of regulation of exocytosis [GO:0017157]; regulates constitutive secretory pathway [GO:0045054] References: PMID:22899725 Sources: GOC:TermGenie, GOC:als, GO_REF:0000058 Subtypes: negative regulation of constitutive secretory pathway [GO:1903434], positive regulation of constitutive secretory pathway [GO:1903435] Definition: Any process that modulates the frequency, rate or extent of constitutive secretory pathway.